urethra epithelium development [GO:0061071] (biological process) Definition: The progression of the urethra epithelium over time from its initial formation to the mature structure. The urethra is a renal system organ that carries urine from the bladder to outside the body. The epithelium is the tubular, planar layer of cells through which the urine passes. Sources: GOC:dph Relationships: is a type of tube development [GO:0035295]; is a type of epithelium development [GO:0060429]; is part of GO:0061068